uropod assembly [GO:0034460] (biological process) Also known as: uropod formation Relationships: is a type of uropod organization [GO:0032796]; is_a plasma membrane bounded cell projection assembly [GO:0120031] Sources: GOC:mah Definition: The assembly of a uropod by rearrangement of the cytoskeleton and overlying membrane.